{
  "gene_name": "A-kinase anchor protein 11",
  "gene_symbol": "AKAP11",
  "term_id": "GO:0007178",
  "term_label": "cell surface receptor protein serine/threonine kinase signaling pathway",
  "gene": "UniProtKB:Q9UKA4"
}